positive regulation of apoptotic process involved in outflow tract morphogenesis [GO:1902258] (biological process) Also known as: up regulation of apoptotic process involved in outflow tract morphogenesis, up-regulation of apoptotic process involved in outflow tract morphogenesis, upregulation of apoptotic process involved in outflow tract morphogenesis, activation of apoptosis involved in outflow tract morphogenesis, activation of apoptotic process involved in outflow tract morphogenesis, positive regulation of apoptosis involved in outflow tract morphogenesis, up regulation of apoptosis involved in outflow tract morphogenesis, up-regulation of apoptosis involved in outflow tract morphogenesis, upregulation of apoptosis involved in outflow tract morphogenesis Definition: Any process that activates or increases the frequency, rate or extent of apoptotic process involved in outflow tract morphogenesis. Relationships: is a type of GO:1902256; is a type of positive regulation of apoptotic process involved in morphogenesis [GO:1902339]; positively regulates apoptotic process involved in outflow tract morphogenesis [GO:0003275] References: PMID:16839542 Sources: GOC:TermGenie, GOC:dph, GOC:mtg_apoptosis